{
  "term_id": "GO:0160072",
  "gene_symbol": "CUL4A",
  "gene": "UniProtKB:Q13619",
  "term_label": "ubiquitin ligase complex scaffold activity",
  "gene_name": "Cullin-4A"
}